{
  "term_id": "UNKNOWN:0002",
  "term_label": "Unknown biological process",
  "gene_name": "Zinc finger protein 474",
  "gene": "UniProtKB:Q6S9Z5",
  "gene_symbol": "ZNF474"
}